{
  "gene_name": "Zinc finger and BTB domain-containing protein 21",
  "term_label": "negative regulation of DNA-templated transcription",
  "gene_symbol": "ZBTB21",
  "gene": "UniProtKB:Q9ULJ3",
  "term_id": "GO:0045892"
}